{
  "term_id": "GO:0007033",
  "term_label": "vacuole organization",
  "gene": "UniProtKB:Q9H270",
  "gene_name": "Vacuolar protein sorting-associated protein 11 homolog",
  "gene_symbol": "VPS11"
}